{
  "gene": "UniProtKB:P05014",
  "gene_name": "Interferon alpha-4",
  "term_id": "GO:0006959",
  "term_label": "humoral immune response",
  "gene_symbol": "IFNA4"
}